subpallium cell proliferation in forebrain [GO:0022012] (biological process) Subtypes: lateral ganglionic eminence cell proliferation [GO:0022018], GO:0022019, GO:0022020, caudal ganglionic eminence cell proliferation [GO:0022021], GO:0022022 Definition: The multiplication or reproduction of subpallium cells in the forebrain, resulting in the expansion of a cell population. Relationships: is a type of cell proliferation in forebrain [GO:0021846]; is part of subpallium development [GO:0021544] Sources: GOC:cls, GOC:dgh, GOC:dph, GOC:jid, GO_REF:0000021